{
  "term_label": "protein localization to plasma membrane",
  "gene": "UniProtKB:Q9BUF7",
  "term_id": "GO:0072659",
  "gene_name": "Protein crumbs homolog 3",
  "gene_symbol": "CRB3"
}